{
  "term_id": "GO:0005737",
  "gene": "UniProtKB:P48723",
  "gene_name": "Heat shock 70 kDa protein 13",
  "gene_symbol": "HSPA13",
  "term_label": "cytoplasm"
}